positive regulation of peptidyl-L-cysteine S-palmitoylation [GO:1902664] (biological process) Also known as: positive regulation of peptidyl-S-palmitoyl-L-cysteine anabolism from peptidyl-cysteine, positive regulation of peptidyl-S-palmitoyl-L-cysteine biosynthetic process from peptidyl-cysteine, positive regulation of peptidyl-S-palmitoyl-L-cysteine formation from peptidyl-cysteine, positive regulation of peptidyl-S-palmitoyl-L-cysteine synthesis from peptidyl-cysteine, positive regulation of peptidyl-cysteine S-palmitoylation, up regulation of peptidyl-L-cysteine S-palmitoylation, up regulation of peptidyl-S-palmitoyl-L-cysteine anabolism from peptidyl-cysteine, up regulation of peptidyl-S-palmitoyl-L-cysteine biosynthetic process from peptidyl-cysteine, up regulation of peptidyl-S-palmitoyl-L-cysteine formation from peptidyl-cysteine, up regulation of peptidyl-S-palmitoyl-L-cysteine synthesis from peptidyl-cysteine, up regulation of peptidyl-cysteine S-palmitoylation, up-regulation of peptidyl-L-cysteine S-palmitoylation, up-regulation of peptidyl-S-palmitoyl-L-cysteine anabolism from peptidyl-cysteine, up-regulation of peptidyl-S-palmitoyl-L-cysteine biosynthetic process from peptidyl-cysteine, up-regulation of peptidyl-S-palmitoyl-L-cysteine formation from peptidyl-cysteine, up-regulation of peptidyl-S-palmitoyl-L-cysteine synthesis from peptidyl-cysteine, up-regulation of peptidyl-cysteine S-palmitoylation, upregulation of peptidyl-L-cysteine S-palmitoylation, upregulation of peptidyl-S-palmitoyl-L-cysteine anabolism from peptidyl-cysteine, upregulation of peptidyl-S-palmitoyl-L-cysteine biosynthetic process from peptidyl-cysteine, upregulation of peptidyl-S-palmitoyl-L-cysteine formation from peptidyl-cysteine, upregulation of peptidyl-S-palmitoyl-L-cysteine synthesis from peptidyl-cysteine, upregulation of peptidyl-cysteine S-palmitoylation, activation of peptidyl-L-cysteine S-palmitoylation, activation of peptidyl-S-palmitoyl-L-cysteine anabolism from peptidyl-cysteine, activation of peptidyl-S-palmitoyl-L-cysteine biosynthetic process from peptidyl-cysteine, activation of peptidyl-S-palmitoyl-L-cysteine formation from peptidyl-cysteine, activation of peptidyl-S-palmitoyl-L-cysteine synthesis from peptidyl-cysteine, activation of peptidyl-cysteine S-palmitoylation Relationships: is a type of GO:1902662; is_a positive regulation of protein lipidation [GO:1903061]; positively regulates peptidyl-L-cysteine S-palmitoylation [GO:0018230] Definition: Any process that activates or increases the frequency, rate or extent of peptidyl-L-cysteine S-palmitoylation. References: PMID:23444136 Sources: GOC:TermGenie, GO_REF:0000058